{
  "gene_symbol": "MRAP2",
  "gene_name": "Melanocortin-2 receptor accessory protein 2",
  "gene": "UniProtKB:Q96G30",
  "term_id": "GO:0005886",
  "term_label": "plasma membrane"
}